negative regulation of type B pancreatic cell apoptotic process [GO:2000675] (biological process) Relationships: is a type of negative regulation of epithelial cell apoptotic process [GO:1904036]; is a type of GO:2000674; negatively regulates GO:0097050 Sources: GOC:mtg_apoptosis, GOC:obol Also known as: negative regulation of pancreatic B cell apoptosis, negative regulation of pancreatic beta cell apoptosis, negative regulation of type B pancreatic cell apoptosis Definition: Any process that stops, prevents or reduces the frequency, rate or extent of type B pancreatic cell apoptotic process.